{
  "gene": "UniProtKB:Q9H201",
  "term_label": "phospholipid binding",
  "term_id": "GO:0005543",
  "gene_symbol": "EPN3",
  "gene_name": "Epsin-3"
}